{
  "term_id": "GO:2000785",
  "gene_symbol": "TBC1D14",
  "gene_name": "TBC1 domain family member 14",
  "gene": "UniProtKB:Q9P2M4",
  "term_label": "regulation of autophagosome assembly"
}